{
  "gene_name": "Keratin, type I cytoskeletal 17",
  "gene_symbol": "KRT17",
  "term_label": "structural constituent of skin epidermis",
  "term_id": "GO:0030280",
  "gene": "UniProtKB:Q04695"
}